{
  "term_id": "UNKNOWN:0002",
  "term_label": "Unknown biological process",
  "gene_name": "Leukocyte surface antigen CD53",
  "gene": "UniProtKB:P19397",
  "gene_symbol": "CD53"
}